wogonin 7-O-glucuronosyltransferase activity [GO:0102468] (molecular function) Definition: Catalysis of the reaction: UDP-alpha-D-glucuronate + wogonin = UDP + wogonin 7-O-beta-D-glucuronate + H+. Sources: RHEA:28322 Relationships: is a type of hexosyltransferase activity [GO:0016758]